mannitol transmembrane transporter activity [GO:0015575] (molecular function) Subtypes: protein-N(PI)-phosphohistidine-mannitol phosphotransferase system transmembrane transporter activity [GO:0022872] Sources: GOC:ai, GOC:mtg_transport, ISBN:0815340729 Definition: Enables the transfer of mannitol from one side of a membrane to the other. Mannitol is the alditol derived from D-mannose by reduction of the aldehyde group. Also known as: mannitol permease activity Relationships: is a type of GO:0015144; is a type of polyol transmembrane transporter activity [GO:0015166]; BFO_0000050 mannitol transmembrane transport [GO:0015797]